{
  "gene_name": "Immunoglobulin lambda variable 8-61",
  "gene_symbol": "IGLV8-61",
  "gene": "UniProtKB:A0A075B6I0",
  "term_label": "Unknown molecular function",
  "term_id": "UNKNOWN:0001"
}